{
  "gene_symbol": "RERG",
  "gene_name": "Ras-related and estrogen-regulated growth inhibitor",
  "term_id": "GO:0007163",
  "term_label": "establishment or maintenance of cell polarity",
  "gene": "UniProtKB:Q96A58"
}